{
  "gene_name": "Peroxisome proliferator-activated receptor gamma",
  "gene": "UniProtKB:P37231",
  "term_label": "positive regulation of fatty acid metabolic process",
  "gene_symbol": "PPARG",
  "term_id": "GO:0045923"
}